{
  "gene_symbol": "KAT6A",
  "term_id": "GO:0010484",
  "term_label": "histone H3 acetyltransferase activity",
  "gene_name": "Histone acetyltransferase KAT6A",
  "gene": "UniProtKB:Q92794"
}